{
  "gene_symbol": "MYLK2",
  "gene_name": "Myosin light chain kinase 2, skeletal_cardiac muscle",
  "term_id": "GO:0006941",
  "term_label": "striated muscle contraction",
  "gene": "UniProtKB:Q9H1R3"
}